{
  "term_id": "GO:0016477",
  "gene_name": "Cadherin-like protein 26",
  "gene_symbol": "CDH26",
  "gene": "UniProtKB:Q8IXH8",
  "term_label": "cell migration"
}